protein localization to polar microtubule [GO:0160086] (biological process) Relationships: is a type of GO:1902889 References: PMID:34080538 Definition: A process in which a protein is transported to, or maintained in, a location within a polar microtubule.